{
  "gene": "UniProtKB:Q9UL15",
  "term_id": "GO:0090083",
  "term_label": "regulation of inclusion body assembly",
  "gene_name": "BAG family molecular chaperone regulator 5",
  "gene_symbol": "BAG5"
}